regulation of oogenesis [GO:1905879] (biological process) References: PMID:26434723 Sources: GOC:TermGenie, GO_REF:0000058 Also known as: regulation of ovum development Relationships: is a type of regulation of multicellular organismal process [GO:0051239]; is a type of regulation of cell development [GO:0060284]; is a type of regulation of reproductive process [GO:2000241]; regulates oogenesis [GO:0048477] Subtypes: regulation of oocyte development [GO:0060281], GO:1905880, positive regulation of oogenesis [GO:1905881] Definition: Any process that modulates the frequency, rate or extent of oogenesis.